{
  "gene_name": "Proteoglycan 3",
  "term_id": "UNKNOWN:0003",
  "gene": "UniProtKB:Q9Y2Y8",
  "gene_symbol": "PRG3",
  "term_label": "Unknown cellular component"
}